{
  "gene_name": "Endosialin",
  "gene": "UniProtKB:Q9HCU0",
  "gene_symbol": "CD248",
  "term_label": "extracellular matrix binding",
  "term_id": "GO:0050840"
}